positive regulation of long-term synaptic potentiation [GO:1900273] (biological process) Sources: GOC:BHF, GOC:TermGenie Relationships: is a type of positive regulation of synaptic transmission [GO:0050806]; is a type of regulation of long-term synaptic potentiation [GO:1900271]; positively regulates long-term synaptic potentiation [GO:0060291] Also known as: activation of long-term potentiation, positive regulation of long-term potentiation, up regulation of long-term potentiation, up-regulation of long-term potentiation, upregulation of long-term potentiation, up regulation of long-term synaptic potentiation, up-regulation of long-term synaptic potentiation, upregulation of long-term synaptic potentiation, activation of long-term synaptic potentiation, activation of LTP, positive regulation of LTP, up regulation of LTP, up-regulation of LTP, upregulation of LTP Definition: Any process that activates or increases the frequency, rate or extent of long-term synaptic potentiation.